endosome organization [GO:0007032] (biological process) Subtypes: GO:0016189, multivesicular body organization [GO:0036257], intralumenal vesicle formation [GO:0070676], endosome membrane tubulation [GO:0097750] Regulation: regulated by regulation of endosome organization [GO:1904978]; negatively regulated by negative regulation of endosome organization [GO:1904979]; RO_0002213 by GO:1904980 Also known as: endosome organisation, endosome organization and biogenesis Sources: GOC:dph, GOC:jl, GOC:mah Definition: A process that is carried out at the cellular level which results in the assembly, arrangement of constituent parts, or disassembly of endosomes. Relationships: is a type of GO:0016050; is part of endomembrane system organization [GO:0010256]